{
  "gene_name": "ATP-dependent RNA helicase DHX8",
  "gene": "UniProtKB:Q14562",
  "term_id": "GO:0071013",
  "term_label": "catalytic step 2 spliceosome",
  "gene_symbol": "DHX8"
}